{
  "term_label": "DNA-binding transcription factor activity, RNA polymerase II-specific",
  "term_id": "GO:0000981",
  "gene": "UniProtKB:Q8NEK5",
  "gene_symbol": "ZNF548",
  "gene_name": "Zinc finger protein 548"
}